{
  "gene_name": "Plexin-D1",
  "gene": "UniProtKB:Q9Y4D7",
  "gene_symbol": "PLXND1",
  "term_id": "GO:0007162",
  "term_label": "negative regulation of cell adhesion"
}